anaerobic 1,1,1-trichloro-2,2-bis-(4-chlorophenyl)ethane metabolic process [GO:0018978] (biological process) Sources: GOC:jl Also known as: anaerobic 1,1,1-trichloro-2,2-bis-(4-chlorophenyl)ethane metabolism, anaerobic DDT metabolic process, anaerobic DDT metabolism Relationships: is a type of GO:0018977 Definition: The chemical reactions and pathways involving 1,1,1-trichloro-2,2-bis-(4-chlorophenyl)ethane (DDT), a chlorinated, broad spectrum, contact insecticide, in the absence of oxygen.